{
  "term_id": "GO:0030198",
  "gene": "UniProtKB:O15072",
  "gene_name": "A disintegrin and metalloproteinase with thrombospondin motifs 3",
  "term_label": "extracellular matrix organization",
  "gene_symbol": "ADAMTS3"
}